gland morphogenesis [GO:0022612] (biological process) Definition: The process in which the anatomical structures of a gland are generated and organized. Relationships: is a type of animal organ morphogenesis [GO:0009887]; BFO_0000050 gland development [GO:0048732] Sources: GOC:isa_complete Subtypes: salivary gland morphogenesis [GO:0007435], neurohypophysis morphogenesis [GO:0048848], hypophysis morphogenesis [GO:0048850], GO:0060443, prostate gland morphogenesis [GO:0060512], seminal vesicle morphogenesis [GO:0061682], liver morphogenesis [GO:0072576]